{
  "term_id": "GO:0005549",
  "gene": "UniProtKB:Q9UGF7",
  "gene_symbol": "OR12D3",
  "term_label": "odorant binding",
  "gene_name": "Olfactory receptor 12D3"
}